{
  "term_id": "GO:0006955",
  "term_label": "immune response",
  "gene_symbol": "IGKV1-33",
  "gene_name": "Immunoglobulin kappa variable 1-33",
  "gene": "UniProtKB:P01594"
}